{
  "term_id": "GO:0005769",
  "gene": "UniProtKB:P51795",
  "term_label": "early endosome",
  "gene_symbol": "CLCN5",
  "gene_name": "H(+)_Cl(-) exchange transporter 5"
}